{
  "gene": "UniProtKB:O75928",
  "gene_name": "E3 SUMO-protein ligase PIAS2",
  "term_label": "protein sumoylation",
  "gene_symbol": "PIAS2",
  "term_id": "GO:0016925"
}